{
  "gene": "UniProtKB:A0A2R8Y4M4",
  "gene_symbol": "LOC122513141",
  "term_label": "protein K63-linked ubiquitination",
  "gene_name": "RING-type domain-containing protein",
  "term_id": "GO:0070534"
}